{
  "gene_name": "A disintegrin and metalloproteinase with thrombospondin motifs 15",
  "term_label": "metalloendopeptidase activity",
  "gene": "UniProtKB:Q8TE58",
  "term_id": "GO:0004222",
  "gene_symbol": "ADAMTS15"
}